{
  "term_id": "GO:0008286",
  "gene_name": "Insulin receptor substrate 1",
  "gene": "UniProtKB:P35568",
  "term_label": "insulin receptor signaling pathway",
  "gene_symbol": "IRS1"
}